negative regulation of cholesterol transport [GO:0032375] (biological process) Also known as: down regulation of cholesterol transport, down-regulation of cholesterol transport, downregulation of cholesterol transport, inhibition of cholesterol transport Sources: GOC:mah Definition: Any process that stops, prevents, or reduces the frequency, rate or extent of the directed movement of cholesterol into, out of or within a cell, or between cells, by means of some agent such as a transporter or pore. Subtypes: negative regulation of intracellular cholesterol transport [GO:0032384], negative regulation of cholesterol import [GO:0060621], negative regulation of cholesterol efflux [GO:0090370], GO:1903063 Relationships: is a type of negative regulation of sterol transport [GO:0032372]; is a type of regulation of cholesterol transport [GO:0032374]; negatively regulates cholesterol transport [GO:0030301]